{
  "term_id": "GO:0005886",
  "gene": "UniProtKB:Q8TDS7",
  "term_label": "plasma membrane",
  "gene_name": "Mas-related G-protein coupled receptor member D",
  "gene_symbol": "MRGPRD"
}